{
  "term_id": "GO:0005730",
  "gene_name": "Protein LLP homolog",
  "term_label": "nucleolus",
  "gene": "UniProtKB:Q9BRT6",
  "gene_symbol": "LLPH"
}